{
  "gene_name": "Ephrin type-A receptor 7",
  "term_id": "GO:0030425",
  "gene_symbol": "EPHA7",
  "gene": "UniProtKB:Q15375",
  "term_label": "dendrite"
}